{
  "gene": "UniProtKB:Q9H2Z4",
  "gene_symbol": "NKX2-4",
  "term_label": "DNA-binding transcription factor activity, RNA polymerase II-specific",
  "term_id": "GO:0000981",
  "gene_name": "Homeobox protein Nkx-2.4"
}